{
  "term_id": "GO:0005765",
  "gene_name": "Natural resistance-associated macrophage protein 1",
  "gene_symbol": "SLC11A1",
  "gene": "UniProtKB:P49279",
  "term_label": "lysosomal membrane"
}